alginic acid acetylation [GO:0051979] (biological process) Also known as: alginate acetylation Relationships: is a type of polysaccharide metabolic process [GO:0005976] Definition: The addition of O-acetyl ester groups to alginic acid, a linear polymer of D-mannuronate and L-guluronate. Sources: GOC:mlg